negative regulation of female pigmentation [GO:0048090] (biological process) Sources: GOC:jid Definition: Any process that stops, prevents, or reduces the frequency, rate or extent of establishment of a pattern of pigment in females. Relationships: is a type of negative regulation of developmental pigmentation [GO:0048086]; is a type of regulation of female pigmentation [GO:0048089]; is a type of negative regulation of developmental process [GO:0051093]; is a type of negative regulation of multicellular organismal process [GO:0051241]; is a type of negative regulation of reproductive process [GO:2000242]; negatively regulates female pigmentation [GO:0048095] Also known as: down regulation of female pigmentation, down-regulation of female pigmentation, downregulation of female pigmentation, inhibition of female pigmentation